{
  "gene": "UniProtKB:Q9BRP4",
  "gene_name": "Proteasomal ATPase-associated factor 1",
  "term_id": "UNKNOWN:0001",
  "gene_symbol": "PAAF1",
  "term_label": "Unknown molecular function"
}